{
  "gene_name": "Putative uncharacterized protein BAALC-AS2",
  "gene_symbol": "BAALC-AS2",
  "term_label": "Unknown cellular component",
  "term_id": "UNKNOWN:0003",
  "gene": "UniProtKB:P0C853"
}